{
  "gene_symbol": "RAB11FIP2",
  "term_id": "GO:0005768",
  "gene": "UniProtKB:Q7L804",
  "term_label": "endosome",
  "gene_name": "Rab11 family-interacting protein 2"
}